{
  "term_label": "cell-cell adhesion",
  "gene": "UniProtKB:Q14126",
  "term_id": "GO:0098609",
  "gene_name": "Desmoglein-2",
  "gene_symbol": "DSG2"
}